{
  "term_label": "Unknown cellular component",
  "gene": "UniProtKB:Q3LI61",
  "gene_name": "Keratin-associated protein 20-2",
  "gene_symbol": "KRTAP20-2",
  "term_id": "UNKNOWN:0003"
}